regulation of gastrin-induced gastric acid secretion [GO:1903639] (biological process) Definition: Any process that modulates the frequency, rate or extent of gastrin-induced gastric acid secretion. Relationships: is a type of GO:0060453; regulates gastrin-induced gastric acid secretion [GO:0001698] References: PMID:11123201 Sources: GOC:TermGenie, GO_REF:0000058 Subtypes: GO:1903640, positive regulation of gastrin-induced gastric acid secretion [GO:1903641]